{
  "gene_name": "Programmed cell death protein 2",
  "gene": "UniProtKB:Q16342",
  "gene_symbol": "PDCD2",
  "term_label": "Unknown molecular function",
  "term_id": "UNKNOWN:0001"
}